apical ectoplasmic specialization [GO:0061831] (cellular component) Also known as: apical ES Relationships: is a type of cell-cell junction [GO:0005911] Definition: Testis-specific junction between mature spermatids and Sertoli cells at the luminal end of the Sertoli cell. References: PMID:22332112, PMID:23546604 Sources: GOC:aruk, GOC:bc, GOC:dph